{
  "term_id": "GO:0007264",
  "gene_name": "GTPase RhebL1",
  "gene": "UniProtKB:Q8TAI7",
  "gene_symbol": "RHEBL1",
  "term_label": "small GTPase-mediated signal transduction"
}